negative regulation of methane biosynthetic process from methanethiol [GO:1900346] (biological process) Definition: Any process that stops, prevents or reduces the frequency, rate or extent of methane biosynthetic process from methanethiol. Relationships: is a type of GO:1900345; is_a negative regulation of alkane biosynthetic process [GO:1901578]; is a type of negative regulation of cellular respiration [GO:1901856]; RO_0002212 methane biosynthetic process from methanethiol [GO:2001133] Also known as: down regulation of methane biosynthetic process from methanethiol, down-regulation of methane biosynthetic process from methanethiol, downregulation of methane biosynthetic process from methanethiol, inhibition of methane biosynthetic process from methanethiol Sources: GOC:TermGenie, GOC:mengo_curators